regulation of dermatome development [GO:0061183] (biological process) Definition: Any process that modulates the rate, frequency, or extent of the progression of the dermatome over time, from its initial formation to the mature structure. The dermatome is the portion of a somite that will form skin. Relationships: is a type of GO:0050793; regulates GO:0061054 Sources: GOC:BHF, GOC:dph Subtypes: positive regulation of dermatome development [GO:0061184], negative regulation of dermatome development [GO:0061185]